{
  "gene_name": "Olfactory receptor 3A2",
  "term_label": "signal transduction",
  "gene_symbol": "OR3A2",
  "gene": "UniProtKB:P47893",
  "term_id": "GO:0007165"
}